{
  "term_label": "external side of plasma membrane",
  "term_id": "GO:0009897",
  "gene": "UniProtKB:P06734",
  "gene_symbol": "FCER2",
  "gene_name": "Low affinity immunoglobulin epsilon Fc receptor"
}